proton transmembrane transport [GO:1902600] (biological process) Relationships: is a type of monoatomic cation transmembrane transport [GO:0098655] Definition: The directed movement of a proton across a membrane. Subtypes: GO:0015985, energy coupled proton transmembrane transport, against electrochemical gradient [GO:0015988], synaptic vesicle lumen acidification [GO:0097401], proton export across plasma membrane [GO:0120029] Also known as: hydrogen transport, proton transport, hydrogen ion transmembrane transport, hydrogen transmembrane transport, ATP hydrolysis coupled proton transport, passive proton transport, down the electrochemical gradient, hydrogen ion transport Sources: GOC:TermGenie, GOC:pr, GO_REF:0000069 Regulation: regulated by GO:0010155